{
  "term_label": "Unknown molecular function",
  "gene_symbol": "KATNBL1",
  "term_id": "UNKNOWN:0001",
  "gene": "UniProtKB:Q9H079",
  "gene_name": "KATNB1-like protein 1"
}